{
  "gene": "UniProtKB:Q9Y4H4",
  "gene_name": "G-protein-signaling modulator 3",
  "term_id": "UNKNOWN:0003",
  "term_label": "Unknown cellular component",
  "gene_symbol": "GPSM3"
}